{
  "gene_name": "Cadherin-5",
  "gene": "UniProtKB:P33151",
  "term_label": "cadherin binding",
  "gene_symbol": "CDH5",
  "term_id": "GO:0045296"
}